{
  "term_id": "GO:0045296",
  "gene_name": "Cadherin-20",
  "gene": "UniProtKB:Q9HBT6",
  "term_label": "cadherin binding",
  "gene_symbol": "CDH20"
}